{
  "term_id": "GO:0000978",
  "term_label": "RNA polymerase II cis-regulatory region sequence-specific DNA binding",
  "gene_name": "Zinc finger protein 444",
  "gene_symbol": "ZNF444",
  "gene": "UniProtKB:Q8N0Y2"
}